{
  "term_id": "GO:0008286",
  "gene_symbol": "GSK3A",
  "gene_name": "Glycogen synthase kinase-3 alpha",
  "gene": "UniProtKB:P49840",
  "term_label": "insulin receptor signaling pathway"
}